positive regulation of barbed-end actin filament capping [GO:2000814] (biological process) Also known as: positive regulation of barbed-end F-actin capping activity, positive regulation of barbed-end actin capping activity, positive regulation of plus-end F-actin capping activity, positive regulation of plus-end actin filament capping activity Relationships: is a type of GO:0051130; is a type of regulation of barbed-end actin filament capping [GO:2000812]; positively regulates barbed-end actin filament capping [GO:0051016] Sources: GOC:BHF Definition: Any process that activates or increases the frequency, rate or extent of barbed-end actin filament capping.